{
  "gene_symbol": "NIT2",
  "gene_name": "Omega-amidase NIT2",
  "term_id": "GO:0006528",
  "term_label": "asparagine metabolic process",
  "gene": "UniProtKB:Q9NQR4"
}